{
  "term_id": "GO:0000978",
  "gene_symbol": "ZNF525",
  "gene_name": "Zinc finger protein 525",
  "gene": "UniProtKB:Q8N782",
  "term_label": "RNA polymerase II cis-regulatory region sequence-specific DNA binding"
}